{
  "gene_name": "Chromosome transmission fidelity protein 8 homolog",
  "term_id": "UNKNOWN:0001",
  "gene": "UniProtKB:P0CG13",
  "term_label": "Unknown molecular function",
  "gene_symbol": "CHTF8"
}